{
  "gene_name": "SH2 domain-containing protein 7",
  "gene_symbol": "SH2D7",
  "gene": "UniProtKB:A6NKC9",
  "term_label": "Unknown biological process",
  "term_id": "UNKNOWN:0002"
}